{
  "gene_name": "Leukosialin",
  "gene": "UniProtKB:P16150",
  "term_id": "GO:0009897",
  "term_label": "external side of plasma membrane",
  "gene_symbol": "SPN"
}